{
  "gene_name": "Large ribosomal subunit protein uL4",
  "term_id": "GO:0003723",
  "term_label": "RNA binding",
  "gene_symbol": "RPL4",
  "gene": "UniProtKB:P36578"
}